{
  "gene": "UniProtKB:Q9H159",
  "gene_name": "Cadherin-19",
  "gene_symbol": "CDH19",
  "term_label": "cadherin binding",
  "term_id": "GO:0045296"
}